{
  "term_id": "GO:0006357",
  "term_label": "regulation of transcription by RNA polymerase II",
  "gene_symbol": "ZNF677",
  "gene_name": "Zinc finger protein 677",
  "gene": "UniProtKB:Q86XU0"
}